{
  "term_id": "GO:0017171",
  "term_label": "serine hydrolase activity",
  "gene_symbol": "AADAC",
  "gene": "UniProtKB:P22760",
  "gene_name": "Arylacetamide deacetylase"
}